negative regulation of establishment of cell polarity regulating cell shape [GO:2000783] (biological process) Relationships: is a type of negative regulation of establishment or maintenance of cell polarity regulating cell shape [GO:2000770]; is a type of GO:2000782; RO_0002212 establishment of cell polarity regulating cell shape [GO:0071964] Definition: Any process that stops, prevents or reduces the frequency, rate or extent of establishment of cell polarity regulating cell shape. Sources: GOC:Mah